{
  "term_id": "GO:0032436",
  "term_label": "positive regulation of proteasomal ubiquitin-dependent protein catabolic process",
  "gene_symbol": "DET1",
  "gene_name": "DET1 homolog",
  "gene": "UniProtKB:Q7L5Y6"
}